{
  "term_label": "cytoplasm",
  "term_id": "GO:0005737",
  "gene": "UniProtKB:P98174",
  "gene_symbol": "FGD1",
  "gene_name": "FYVE, RhoGEF and PH domain-containing protein 1"
}